S-acetyltransferase activity [GO:0016418] (molecular function) Sources: GOC:ai Subtypes: [acyl-carrier-protein] S-acetyltransferase activity [GO:0004313], dihydrolipoyllysine-residue acetyltransferase activity [GO:0004742], deacetyl-[citrate-(pro-3S)-lyase] S-acetyltransferase activity [GO:0047187], hydrogen-sulfide S-acetyltransferase activity [GO:0047986], GO:0050336 Relationships: is a type of GO:0016407; is_a GO:0016417 Definition: Catalysis of the transfer of an acetyl group to a sulfur atom on the acceptor molecule.